dCTP diphosphatase activity [GO:0047840] (molecular function) Definition: Catalysis of the reaction: dCTP + H2O = dCMP + H+ + diphosphate. Also known as: dCTP pyrophosphatase activity, dCTP nucleotidohydrolase activity, dCTPase activity, deoxy-CTPase activity, deoxycytidine triphosphatase activity, deoxycytidine-triphosphatase activity Sources: RHEA:22636 Relationships: is_a nucleoside triphosphate diphosphatase activity [GO:0047429]